regulation of tyramine signaling pathway [GO:2000131] (biological process) Also known as: regulation of tyramine signalling pathway Definition: Any process that modulates the frequency, rate or extent of tyramine signaling pathway. Subtypes: negative regulation of tyramine signaling pathway [GO:2000132], positive regulation of tyramine signaling pathway [GO:2000133] Relationships: is a type of regulation of octopamine or tyramine signaling pathway [GO:2000125]; regulates GO:0071928 Sources: GOC:mah